{
  "term_label": "innate immune response",
  "gene_name": "Shiftless antiviral inhibitor of ribosomal frameshifting protein",
  "gene_symbol": "SHFL",
  "term_id": "GO:0045087",
  "gene": "UniProtKB:Q9NUL5"
}